chemoattraction involved in embryonic olfactory bulb interneuron precursor migration [GO:0021835] (biological process) Definition: The creation and reception of signals that result in the migration of interneuron precursors up a concentration gradient towards the olfactory bulb. References: PMID:12626695 Sources: GOC:cls, GOC:dgh, GOC:dph, GOC:jid, GO_REF:0000021 Also known as: positive chemotaxis involved in embryonic olfactory bulb interneuron precursor migration Relationships: is a type of positive chemotaxis [GO:0050918]; is part of embryonic olfactory bulb interneuron precursor migration [GO:0021831]